{
  "term_id": "GO:0050727",
  "gene": "UniProtKB:Q7RTR0",
  "term_label": "regulation of inflammatory response",
  "gene_symbol": "NLRP9",
  "gene_name": "NACHT, LRR and PYD domains-containing protein 9"
}